positive regulation of chaperone-mediated autophagy [GO:1904716] (biological process) Relationships: is a type of positive regulation of autophagy [GO:0010508]; is a type of positive regulation of protein catabolic process [GO:0045732]; is a type of regulation of chaperone-mediated autophagy [GO:1904714]; positively regulates chaperone-mediated autophagy [GO:0061684] Also known as: up regulation of chaperone-mediated autophagy, up-regulation of chaperone-mediated autophagy, upregulation of chaperone-mediated autophagy, activation of chaperone-mediated autophagy, activation of CMA, positive regulation of CMA, up regulation of CMA, up-regulation of CMA, upregulation of CMA Definition: Any process that activates or increases the frequency, rate or extent of chaperone-mediated protein folding. References: PMID:24375412